negative regulation of platelet-derived growth factor receptor-alpha signaling pathway [GO:2000584] (BP) Also known as: negative regulation of PDGF receptor-alpha signaling pathway, negative regulation of alphaPDGF receptor signaling pathway, negative regulation of platelet-derived growth factor receptor-alpha signalling pathway, negative regulation of PDGFR-alpha signaling pathway Sources: GOC:obol, GOC:yaf Definition: Any process that stops, prevents or reduces the frequency, rate or extent of platelet-derived growth factor receptor-alpha signaling pathway. Relationships: is a type of GO:0010642; is a type of regulation of platelet-derived growth factor receptor-alpha signaling pathway [GO:2000583]; negatively regulates platelet-derived growth factor receptor-alpha signaling pathway [GO:0035790]